{
  "term_label": "mitochondrial inner membrane",
  "term_id": "GO:0005743",
  "gene_name": "OCIA domain-containing protein 2",
  "gene_symbol": "OCIAD2",
  "gene": "UniProtKB:Q56VL3"
}